oospore formation [GO:0075243] (biological process) Regulation: regulated by regulation of oospore formation [GO:0075244]; positively regulated by positive regulation of oospore formation [GO:0075245]; negatively regulated by negative regulation of oospore formation [GO:0075246] Relationships: is a type of sexual sporulation resulting in formation of a cellular spore [GO:0043935] Sources: GOC:pamgo_curators Definition: The process in which male and female gametangia develop and fuse to form an oospore, a thick-walled resting spore of Oomycetes and certain algae and fungi.